{
  "gene": "UniProtKB:O75333",
  "gene_symbol": "TBX10",
  "gene_name": "T-box transcription factor TBX10",
  "term_label": "RNA polymerase II cis-regulatory region sequence-specific DNA binding",
  "term_id": "GO:0000978"
}